{
  "gene_symbol": "CYLD",
  "term_label": "cysteine-type deubiquitinase activity",
  "gene": "UniProtKB:Q9NQC7",
  "term_id": "GO:0004843",
  "gene_name": "Ubiquitin carboxyl-terminal hydrolase CYLD"
}